{
  "term_id": "GO:0005654",
  "gene_name": "E3 ubiquitin-protein ligase TRIM21",
  "term_label": "nucleoplasm",
  "gene_symbol": "TRIM21",
  "gene": "UniProtKB:P19474"
}